{
  "gene_name": "1-phosphatidylinositol 3-phosphate 5-kinase",
  "gene_symbol": "PIKFYVE",
  "gene": "UniProtKB:Q9Y2I7",
  "term_label": "neutrophil chemotaxis",
  "term_id": "GO:0030593"
}